{
  "gene_symbol": "SYNM",
  "gene": "UniProtKB:O15061",
  "term_id": "GO:0060053",
  "gene_name": "Synemin",
  "term_label": "neurofilament cytoskeleton"
}